{
  "gene_name": "7SK snRNA methylphosphate capping enzyme",
  "term_id": "GO:0017069",
  "gene": "UniProtKB:Q7L2J0",
  "gene_symbol": "MEPCE",
  "term_label": "snRNA binding"
}